{
  "term_id": "GO:0006086",
  "gene_symbol": "PDHB",
  "term_label": "pyruvate decarboxylation to acetyl-CoA",
  "gene_name": "Pyruvate dehydrogenase E1 component subunit beta, mitochondrial",
  "gene": "UniProtKB:P11177"
}